mesonephric duct development [GO:0072177] (biological process) Also known as: Wolffian duct development Relationships: is a type of GO:0072164; is_a GO:0072176 Sources: GOC:mtg_kidney_jan10 Definition: The process whose specific outcome is the progression of a mesonephric duct over time, from its initial formation to a mature structure. A mesonephric duct is a tube drains the mesonephros.